negative regulation of trichoblast fate specification [GO:0010062] (biological process) Definition: Any process that suppresses trichoblast fate specification. Sources: GOC:tb Also known as: down regulation of trichoblast fate, down-regulation of trichoblast fate, downregulation of trichoblast fate, inhibition of trichoblast fate Relationships: is a type of negative regulation of cell fate specification [GO:0009996]; is a type of regulation of trichoblast fate specification [GO:0010061]; is_a negative regulation of plant epidermal cell differentiation [GO:1903889]; RO_0002212 trichoblast fate specification [GO:0010057]